{
  "gene": "UniProtKB:P21796",
  "term_id": "GO:0005741",
  "gene_name": "Voltage-dependent anion-selective channel protein 1",
  "gene_symbol": "VDAC1",
  "term_label": "mitochondrial outer membrane"
}